{
  "gene_symbol": "IL17RE",
  "gene": "UniProtKB:Q8NFR9",
  "term_id": "UNKNOWN:0003",
  "term_label": "Unknown cellular component",
  "gene_name": "Interleukin-17 receptor E"
}